{
  "gene_symbol": "SH3KBP1",
  "term_id": "GO:0030674",
  "gene": "UniProtKB:Q96B97",
  "gene_name": "SH3 domain-containing kinase-binding protein 1",
  "term_label": "protein-macromolecule adaptor activity"
}